{
  "gene": "UniProtKB:Q8N3T1",
  "term_id": "GO:0006493",
  "term_label": "protein O-linked glycosylation",
  "gene_name": "Polypeptide N-acetylgalactosaminyltransferase 15",
  "gene_symbol": "GALNT15"
}